{
  "gene_name": "Matrilysin",
  "gene": "UniProtKB:P09237",
  "term_id": "GO:0030198",
  "gene_symbol": "MMP7",
  "term_label": "extracellular matrix organization"
}